mature follicle stage [GO:0048166] (biological process) Definition: The stage in oogenesis when the antrum is swollen with follicular fluid. The ovum is ready to erupt from the ovary and is arrested at metaphase of the second meiotic division. Sources: GOC:jid, GOC:mtg_sensu, ISBN:0198542771 Relationships: is a type of mammalian oogenesis stage [GO:0022605] Also known as: mammalian oogenesis stage 9